{
  "term_label": "mRNA 3'-UTR binding",
  "gene_symbol": "LARP4",
  "gene": "UniProtKB:Q71RC2",
  "gene_name": "La-related protein 4",
  "term_id": "GO:0003730"
}